response to lipid [GO:0033993] (biological process) Sources: GOC:sl Subtypes: response to lipid hydroperoxide [GO:0006982], response to abscisic acid [GO:0009737], GO:0009739, response to brassinosteroid [GO:0009741], response to estradiol [GO:0032355], response to lipopolysaccharide [GO:0032496], response to retinoic acid [GO:0032526], response to vitamin A [GO:0033189], response to vitamin D [GO:0033280], response to testosterone [GO:0033574], response to triglyceride [GO:0034014], response to prostaglandin [GO:0034694], GO:0036314, GO:0048545, response to fatty acid [GO:0070542], cellular response to lipid [GO:0071396], response to papulacandin B [GO:0072730], response to farnesol [GO:0097307], response to ceramide [GO:0106096], response to butan-1-ol [GO:1901422], response to propan-1-ol [GO:1901427], response to strigolactone [GO:1902347], GO:1903412, GO:1903491, response to dehydroepiandrosterone [GO:1903494], response to micafungin [GO:1903967], GO:1904316, response to forskolin [GO:1904321], response to 1-oleoyl-sn-glycerol 3-phosphate [GO:1904565], response to phorbol 13-acetate 12-myristate [GO:1904627], GO:1904629, response to astaxanthin [GO:1905217], GO:1905230, response to beta-carotene [GO:1905387], GO:1905711, GO:1905836 Relationships: is a type of GO:0042221 Definition: Any process that results in a change in state or activity of a cell or an organism (in terms of movement, secretion, enzyme production, gene expression, etc.) as a result of a lipid stimulus.